{
  "term_id": "GO:0006366",
  "gene_symbol": "POLR2E",
  "gene": "UniProtKB:P19388",
  "gene_name": "DNA-directed RNA polymerases I, II, and III subunit RPABC1",
  "term_label": "transcription by RNA polymerase II"
}